{
  "term_label": "CRD-mediated mRNA stabilization",
  "term_id": "GO:0070934",
  "gene_name": "Insulin-like growth factor 2 mRNA-binding protein 1",
  "gene": "UniProtKB:Q9NZI8",
  "gene_symbol": "IGF2BP1"
}